{
  "term_id": "GO:0043186",
  "gene_symbol": "PIWIL3",
  "term_label": "P granule",
  "gene_name": "Piwi-like protein 3",
  "gene": "UniProtKB:Q7Z3Z3"
}